negative regulation of bacterial-type flagellum assembly [GO:1902209] (biological process) Sources: GOC:TermGenie, GOC:jl Also known as: down regulation of bacterial flagellum assembly, down regulation of bacterial-type flagellum assembly, down-regulation of bacterial flagellum assembly, down-regulation of bacterial-type flagellum assembly, downregulation of bacterial flagellum assembly, downregulation of bacterial-type flagellum assembly, negative regulation of bacterial flagellum assembly, inhibition of bacterial flagellum assembly, inhibition of bacterial-type flagellum assembly Relationships: is a type of negative regulation of cell projection organization [GO:0031345]; is a type of negative regulation of organelle assembly [GO:1902116]; is a type of regulation of bacterial-type flagellum assembly [GO:1902208]; negatively regulates bacterial-type flagellum assembly [GO:0044780] Definition: Any process that stops, prevents or reduces the frequency, rate or extent of bacterial-type flagellum assembly.